{
  "gene_name": "Polypeptide N-acetylgalactosaminyltransferase 3",
  "term_label": "polypeptide N-acetylgalactosaminyltransferase activity",
  "gene": "UniProtKB:Q14435",
  "gene_symbol": "GALNT3",
  "term_id": "GO:0004653"
}